{
  "gene_symbol": "COBLL1",
  "term_id": "UNKNOWN:0002",
  "gene": "UniProtKB:Q53SF7",
  "term_label": "Unknown biological process",
  "gene_name": "Cordon-bleu protein-like 1"
}